{
  "gene_symbol": "CD1D",
  "term_id": "GO:0071723",
  "term_label": "lipopeptide binding",
  "gene": "UniProtKB:P15813",
  "gene_name": "Antigen-presenting glycoprotein CD1d"
}